adult salivary gland boundary specification [GO:0007434] (biological process) Also known as: larval salivary gland determination References: PMID:11598957 Sources: GOC:tb Regulation: regulated by regulation of adult salivary gland boundary specification [GO:0045707]; negatively regulated by GO:0045709; positively regulated by GO:0045711 Definition: Determination in an adult organism of where the salivary gland forms, the total number of salivary gland cells and how many cells are allocated to each of the specialised cell types within the salivary gland. Relationships: is a type of GO:0007432